{
  "gene": "UniProtKB:Q8NGI1",
  "gene_name": "Putative olfactory receptor 56B2",
  "term_id": "UNKNOWN:0002",
  "term_label": "Unknown biological process",
  "gene_symbol": "OR56B2"
}